{
  "term_id": "UNKNOWN:0001",
  "gene": "UniProtKB:A6NKN8",
  "term_label": "Unknown molecular function",
  "gene_symbol": "PCP4L1",
  "gene_name": "Purkinje cell protein 4-like protein 1"
}